{
  "gene_symbol": "PAK2",
  "term_id": "GO:0009267",
  "gene_name": "Serine_threonine-protein kinase PAK 2",
  "gene": "UniProtKB:Q13177",
  "term_label": "cellular response to starvation"
}